{
  "gene_name": "Guanine nucleotide-binding protein subunit alpha-13",
  "term_id": "GO:0003924",
  "gene": "UniProtKB:Q14344",
  "term_label": "GTPase activity",
  "gene_symbol": "GNA13"
}